{
  "gene_name": "Trifunctional purine biosynthetic protein adenosine-3",
  "gene_symbol": "GART",
  "term_label": "phosphoribosylformylglycinamidine cyclo-ligase activity",
  "gene": "UniProtKB:P22102",
  "term_id": "GO:0004641"
}